{
  "gene_symbol": "IL21",
  "term_label": "positive regulation of natural killer cell mediated cytotoxicity",
  "gene_name": "Interleukin-21",
  "gene": "UniProtKB:Q9HBE4",
  "term_id": "GO:0045954"
}